G protein-coupled glycine receptor activity [GO:0160079] (molecular function) Definition: Combining with glycine and transmitting the signal across the membrane by changing the activity of intracellular G protein signaling. References: PMID:36996198 Also known as: mGlyR, metabotropic glycine receptor activity Relationships: is a type of G protein-coupled neurotransmitter receptor activity [GO:0099528]